{
  "term_id": "GO:0045130",
  "term_label": "keratan sulfotransferase activity",
  "gene_symbol": "CHST1",
  "gene": "UniProtKB:O43916",
  "gene_name": "Carbohydrate sulfotransferase 1"
}